{
  "term_label": "regulation of transcription by RNA polymerase II",
  "gene_name": "Highly divergent homeobox",
  "gene": "UniProtKB:Q7Z353",
  "gene_symbol": "HDX",
  "term_id": "GO:0006357"
}